{
  "term_id": "GO:0016485",
  "gene_symbol": "PCSK7",
  "gene_name": "Proprotein convertase subtilisin_kexin type 7",
  "gene": "UniProtKB:Q16549",
  "term_label": "protein processing"
}